{
  "gene_name": "Centromere protein V-like protein 1",
  "term_id": "UNKNOWN:0002",
  "term_label": "Unknown biological process",
  "gene_symbol": "CENPVL1",
  "gene": "UniProtKB:A0A0U1RR11"
}